{
  "gene": "UniProtKB:Q9UBV2",
  "gene_symbol": "SEL1L",
  "term_label": "ERAD pathway",
  "gene_name": "Protein sel-1 homolog 1",
  "term_id": "GO:0036503"
}